{
  "term_id": "UNKNOWN:0002",
  "gene": "UniProtKB:A6ND48",
  "gene_name": "Olfactory receptor 14I1",
  "gene_symbol": "OR14I1",
  "term_label": "Unknown biological process"
}